symbiont defense to host-produced reactive oxygen species [GO:0052164] (biological process) Definition: A process in which a symbiont alters or subverts either the host signal transduction pathways leading to the production of reactive oxygen species as part of the host innate immune response. Relationships: is a type of cellular response to oxidative stress [GO:0034599]; is a type of GO:0052167 Subtypes: GO:0033661, symbiont-mediated detoxification of host-generated reactive oxygen species [GO:0141082] Sources: GOC:mtg_pamgo_17jul06 Also known as: evasion or tolerance by organism of reactive oxygen species produced by other organism involved in symbiotic interaction, evasion or tolerance by symbiont of reactive oxygen species produced by other organism involved in symbiotic interaction, modulation by organism of defense-related reactive oxygen species production in other organism involved in symbiotic interaction, response to defense-related reactive oxygen species production by other organism involved in symbiotic interaction, evasion or tolerance by organism of host-produced reactive oxygen species, evasion or tolerance by organism of reactive oxygen species produced during host defense response, evasion or tolerance by symbiont of host-produced reactive oxygen species, evasion or tolerance of defense-related host metabolic burst, evasion or tolerance of defense-related host oxidative burst, evasion or tolerance of defense-related host respiratory burst, evasion or tolerance of host-produced AOS, evasion or tolerance of host-produced ROIs, evasion or tolerance of host-produced ROS, evasion or tolerance of host-produced active oxygen species, evasion or tolerance of host-produced reactive oxygen intermediates, evasion or tolerance of reactive oxygen species produced by host, modulation by organism of defense-related host AOS production, modulation by organism of defense-related host ROI production, modulation by organism of defense-related host ROS production, modulation by organism of defense-related host active oxygen species production, modulation by organism of defense-related host metabolic burst, modulation by organism of defense-related host oxidative burst, modulation by organism of defense-related host reactive oxidative species production, modulation by organism of defense-related host reactive oxygen intermediate production, modulation by organism of defense-related host respiratory burst, evasion by symbiont of cellular damage caused by host oxidative burst, modulation by symbiont of defense-related host reactive oxygen species production, response to defense-related host reactive oxygen species production